4-hydroxybenzoate 3-monooxygenase (NADH) activity [GO:0106355] (molecular function) Definition: Catalysis of the reaction: 4-hydroxybenzoate + H+ + NADH + O2 = 3,4-dihydroxybenzoate + H2O + NAD+. Sources: RHEA:19473 Relationships: is a type of 4-hydroxybenzoate 3-monooxygenase [NAD(P)H] activity [GO:0018671]